{
  "gene": "UniProtKB:O75791",
  "term_label": "cytoplasm",
  "term_id": "GO:0005737",
  "gene_symbol": "GRAP2",
  "gene_name": "GRB2-related adapter protein 2"
}